{
  "term_label": "calcium ion binding",
  "term_id": "GO:0005509",
  "gene_symbol": "PLA2G4F",
  "gene_name": "Cytosolic phospholipase A2 zeta",
  "gene": "UniProtKB:Q68DD2"
}